{
  "gene_name": "B-cell CLL_lymphoma 9-like protein",
  "term_label": "negative regulation of transforming growth factor beta receptor signaling pathway",
  "gene_symbol": "BCL9L",
  "term_id": "GO:0030512",
  "gene": "UniProtKB:Q86UU0"
}